{
  "term_id": "UNKNOWN:0002",
  "gene": "UniProtKB:Q86X53",
  "gene_name": "Glutamate-rich protein 1",
  "gene_symbol": "ERICH1",
  "term_label": "Unknown biological process"
}